cell cycle checkpoint signaling [GO:0000075] (biological process) Regulation: regulated by regulation of cell cycle checkpoint [GO:1901976]; negatively regulated by negative regulation of cell cycle checkpoint [GO:1901977]; RO_0002213 by GO:1901978 Also known as: cell cycle checkpoint, signal transduction involved in G2/M transition checkpoint, signal transduction involved in cell cycle checkpoint, G1/S checkpoint, G1/S transition checkpoint, G2/M checkpoint, G2/M transition checkpoint Note: This term should not be used in direct manual annotation as it should always be possible to minimally designate mitotic or meiotic checkpoint, and usually to additionally specify the checkpoint (i.e mitotic spindle assembly checkpoint, mitotic DNA damage checkpoint etc). Note also that the effector processes are not part of the checkpoint but are positively regulated by the checkpoint signaling and should not be annotated here. Sources: GOC:mtg_cell_cycle Relationships: is a type of intracellular signal transduction [GO:0035556]; is a type of negative regulation of cell cycle phase transition [GO:1901988] Definition: A signaling process that controls cell cycle progression by monitoring the integrity of specific cell cycle events. A cell cycle checkpoint begins with detection of deficiencies or defects and ends with signal transduction. Subtypes: GO:0007093, GO:0031570, spindle checkpoint signaling [GO:0031577], meiotic cell cycle checkpoint signaling [GO:0033313]